{
  "term_label": "GTPase activity",
  "gene": "UniProtKB:P09471",
  "term_id": "GO:0003924",
  "gene_symbol": "GNAO1",
  "gene_name": "Guanine nucleotide-binding protein G(o) subunit alpha"
}